{
  "term_id": "GO:0005737",
  "gene": "UniProtKB:Q9H4B7",
  "term_label": "cytoplasm",
  "gene_symbol": "TUBB1",
  "gene_name": "Tubulin beta-1 chain"
}